{
  "term_id": "UNKNOWN:0001",
  "gene_symbol": "PLIN4",
  "term_label": "Unknown molecular function",
  "gene": "UniProtKB:Q96Q06",
  "gene_name": "Perilipin-4"
}